{
  "gene_name": "Heterogeneous nuclear ribonucleoprotein H3",
  "gene_symbol": "HNRNPH3",
  "gene": "UniProtKB:P31942",
  "term_label": "regulation of RNA splicing",
  "term_id": "GO:0043484"
}